cholate 7-alpha-dehydrogenase (NAD+) activity [GO:0008709] (MF) Relationships: is a type of steroid dehydrogenase activity, acting on the CH-OH group of donors, NAD or NADP as acceptor [GO:0033764] Sources: RHEA:19409 Also known as: 7-alpha-hydroxysteroid dehydrogenase activity, 7alpha-hydroxy steroid dehydrogenase activity, 7alpha-hydroxysteroid dehydrogenase activity, 7alpha-hydroxysteroid:NAD+ 7-oxidoreductase activity, 7alpha-HSDH Definition: Catalysis of the reaction: cholate + NAD+ = -3alpha,12-alpha-dihydroxy-7-oxo--5beta-cholanate + H+ + NADH.